{
  "gene": "UniProtKB:P11831",
  "term_id": "GO:0045944",
  "gene_symbol": "SRF",
  "term_label": "positive regulation of transcription by RNA polymerase II",
  "gene_name": "Serum response factor"
}